{
  "term_id": "GO:0000976",
  "gene_name": "Forkhead box protein N1",
  "term_label": "transcription cis-regulatory region binding",
  "gene": "UniProtKB:O15353",
  "gene_symbol": "FOXN1"
}